Lands organization [GO:0030577] (biological process) References: PMID:10921892, PMID:8695863 Sources: GOC:mah Also known as: LYSP100-associated nuclear domain organization, Lands organisation, Lands organization and biogenesis Definition: A process that is carried out at the cellular level which results in the assembly, arrangement of constituent parts, or disassembly of Lands, a class of nuclear body that react against SP140 auto-antibodies. Relationships: is a type of GO:0030575 Note: See also the cellular component term 'Lands ; GO:0016606'.